ferric-enterobactin transmembrane transporter activity [GO:0015620] (molecular function) Sources: GOC:ai Relationships: is a type of siderophore-iron transmembrane transporter activity [GO:0015343]; is part of ferric-enterobactin import into cell [GO:0015685] Definition: Enables the transfer of ferric-enterobactin from one side of a membrane to the other.